{
  "term_id": "GO:0006391",
  "gene_symbol": "TFAM",
  "gene_name": "Transcription factor A, mitochondrial",
  "gene": "UniProtKB:Q00059",
  "term_label": "transcription initiation at mitochondrial promoter"
}